{
  "gene_symbol": "KRT87P",
  "gene_name": "Putative keratin-87 protein",
  "gene": "UniProtKB:A6NCN2",
  "term_label": "Unknown molecular function",
  "term_id": "UNKNOWN:0001"
}